{
  "gene_name": "Solute carrier family 12 member 2",
  "term_id": "GO:0016324",
  "gene_symbol": "SLC12A2",
  "gene": "UniProtKB:P55011",
  "term_label": "apical plasma membrane"
}